{
  "gene_symbol": "C8orf90",
  "gene_name": "Uncharacterized protein C8orf90",
  "gene": "UniProtKB:A0A2R8Y2Y2",
  "term_label": "Unknown cellular component",
  "term_id": "UNKNOWN:0003"
}